{
  "gene": "UniProtKB:Q8IWT6",
  "term_label": "cyclic-GMP-AMP transmembrane import across plasma membrane",
  "term_id": "GO:0140361",
  "gene_name": "Volume-regulated anion channel subunit LRRC8A",
  "gene_symbol": "LRRC8A"
}